{
  "gene_symbol": "SPMAP2",
  "gene_name": "Testicular haploid expressed gene protein",
  "term_id": "UNKNOWN:0001",
  "gene": "UniProtKB:Q9P2T0",
  "term_label": "Unknown molecular function"
}